{
  "gene": "UniProtKB:Q9NZI6",
  "term_label": "DNA-binding transcription activator activity, RNA polymerase II-specific",
  "gene_symbol": "TFCP2L1",
  "gene_name": "Transcription factor CP2-like protein 1",
  "term_id": "GO:0001228"
}